{
  "gene_name": "Galectin-3",
  "gene_symbol": "LGALS3",
  "term_label": "laminin binding",
  "term_id": "GO:0043236",
  "gene": "UniProtKB:P17931"
}